2-haloacid dehalogenase (configuration-inverting) activity [GO:0033976] (molecular function) Also known as: 2-haloalkanoic acid dehalogenase activity, 2-haloalkanoid acid halidohydrolase activity, DL-2-haloacid dehalogenase activity, DL-2-haloacid dehalogenase (inversion of configuration) activity, DL-2-haloacid halidohydrolase (inversion of configuration) activity, DL-DEXi Definition: Catalysis of the reactions: an (S)-2-haloacid + H2O = a (2R)-2-hydroxycarboxylate + a halide anion + H+, and an (R)-2-haloacid + H2O = a (2S)-2-hydroxycarboxylate + a halide anion + H+. Sources: EC:3.8.1.10 Relationships: is a type of hydrolase activity, acting on acid halide bonds, in C-halide compounds [GO:0019120]